positive regulation of lipid biosynthetic process [GO:0046889] (biological process) Also known as: positive regulation of lipid anabolism, positive regulation of lipid biosynthesis, positive regulation of lipid formation, positive regulation of lipid synthesis, positive regulation of lipogenesis, up regulation of lipid biosynthetic process, up-regulation of lipid biosynthetic process, upregulation of lipid biosynthetic process, activation of lipid biosynthetic process, stimulation of lipid biosynthetic process Subtypes: positive regulation of abscisic acid biosynthetic process [GO:0010116], GO:0010372, positive regulation of triglyceride biosynthetic process [GO:0010867], GO:0010893, positive regulation of fatty acid biosynthetic process [GO:0045723], positive regulation of juvenile hormone biosynthetic process [GO:0045969], positive regulation of phospholipid biosynthetic process [GO:0071073], GO:0090154, GO:0140736, positive regulation of retinoic acid biosynthetic process [GO:1900054], GO:1900482, positive regulation of butyryl-CoA catabolic process to butanol [GO:1900499], positive regulation of emericellamide biosynthetic process [GO:1900660], positive regulation of isoprene biosynthetic process [GO:1900949], GO:1901544, positive regulation of carotenoid biosynthetic process [GO:1904143], GO:1904278, positive regulation of phytol biosynthetic process [GO:1904964] Sources: GOC:ai Definition: Any process that activates or increases the frequency, rate or extent of the chemical reactions and pathways resulting in the formation of lipids. Relationships: is a type of positive regulation of biosynthetic process [GO:0009891]; is a type of positive regulation of lipid metabolic process [GO:0045834]; is a type of regulation of lipid biosynthetic process [GO:0046890]; positively regulates lipid biosynthetic process [GO:0008610]